{
  "gene_symbol": "NRAP",
  "term_id": "GO:0051015",
  "term_label": "actin filament binding",
  "gene_name": "Nebulin-related-anchoring protein",
  "gene": "UniProtKB:Q86VF7"
}